protocadherin-alpha-v7-protocadherin-gamma-a3 complex [GO:0071189] (cellular component) Also known as: Pcdha7-Pcdhga3 complex Definition: A protein complex that contains the cell adhesion molecules protocadherin-alpha-v7 and protocadherin-gamma-a3, and is involved in the regulation of protein localization to the plasma membrane. References: PMID:15347688 Relationships: is a type of protocadherin-alpha-protocadherin-gamma complex [GO:0071183]